skotomorphogenesis [GO:0009647] (biological process) Also known as: etiolation Relationships: is a type of response to absence of light [GO:0009646]; is a type of GO:0009791 References: PMID:15012288 Definition: The control of plant growth, development, and differentiation in response to growth in darkness.